{
  "gene_symbol": "NCBP2",
  "gene": "UniProtKB:P52298",
  "gene_name": "Nuclear cap-binding protein subunit 2",
  "term_id": "GO:0000398",
  "term_label": "mRNA splicing, via spliceosome"
}